fucose transmembrane transport [GO:0015756] (biological process) Also known as: fucose transport Sources: GOC:ai Relationships: is a type of hexose transmembrane transport [GO:0008645] Definition: The process in which fucose is transported across a lipid bilayer, from one side of a membrane to the other. Fucose is 6-deoxygalactose and has two enantiomers, D-fucose and L-fucose.